{
  "gene_symbol": "BOLL",
  "gene_name": "Protein boule-like",
  "term_id": "GO:0008494",
  "gene": "UniProtKB:Q8N9W6",
  "term_label": "translation activator activity"
}